{
  "gene_name": "Amyloid beta precursor like protein 1",
  "gene_symbol": "APLP1",
  "term_id": "GO:0031694",
  "gene": "UniProtKB:P51693",
  "term_label": "alpha-2A adrenergic receptor binding"
}